reactive gliosis [GO:0150103] (BP) References: PMID:24462092 Sources: GOC:aruk, GOC:bc Relationships: is a type of neuroinflammatory response [GO:0150076] Also known as: gliosis Definition: A neuroinflammatory response, occurring over several days, during which glial cells undergo nonspecific reactive changes in response to damage to the central nervous system (CNS); typically involves the proliferation or hypertrophy of different types of glial cells.